{
  "term_label": "calcium ion export across plasma membrane",
  "gene": "UniProtKB:P57103",
  "term_id": "GO:1990034",
  "gene_name": "Sodium_calcium exchanger 3",
  "gene_symbol": "SLC8A3"
}